GDP-Man:Man(3)GlcNAc(2)-PP-Dol alpha-1,2-mannosyltransferase activity [GO:0004377] (molecular function) Definition: Catalysis of the reaction: an alpha-D-Man-(1->3)-[alpha-D-Man-(1->6)]-beta-D-Man-(1->4)-beta-D-GlcNAc-(1->4)-alpha-D-GlcNAc-diphospho-di-trans,poly-cis-dolichol + 2 GDP-alpha-D-mannose = an alpha-D-Man-(1->2)-alpha-D-Man-(1->2)-alpha-D-Man-(1->3)-[alpha-D-Man-(1->6)]-beta-D-Man-(1->4)-beta-D-GlcNAc-(1->4)-alpha-D-GlcNAc-diphospho-di-trans,poly-cis-dolichol + 2 GDP + 2 H+. Sources: RHEA:29523 Relationships: is a type of alpha-1,2-mannosyltransferase activity [GO:0000026]; is_a GlcNAc(2)-PP-Dol mannosyltransferase activity [GO:0120562] Also known as: GDP-D-mannose:D-Man-alpha-(1->3)-[D-Man-alpha-(1->6)]-D-Man-beta-(1->4)-D-GlcNAc-beta-(1->4)-D-GlcNAc-diphosphodolichol alpha-1,2-mannosyltransferase activity, GDP-mannose-oligosaccharide-lipid mannosyltransferase activity, GDP-mannose:glycolipid 1,2-alpha-D-mannosyltransferase activity, glycolipid 2-alpha-mannosyltransferase activity, guanosine diphosphomannose-oligosaccharide-lipid mannosyltransferase activity, oligosaccharide-lipid mannosyltransferase activity